{
  "gene": "UniProtKB:P27701",
  "gene_symbol": "CD82",
  "term_label": "Unknown molecular function",
  "term_id": "UNKNOWN:0001",
  "gene_name": "CD82 antigen"
}